{
  "gene": "UniProtKB:Q92503",
  "gene_symbol": "SEC14L1",
  "gene_name": "SEC14-like protein 1",
  "term_id": "GO:0039536",
  "term_label": "negative regulation of RIG-I signaling pathway"
}